box C/D pre-rRNA cleavage RNP complex [GO:0170052] (cellular component) Definition: A ribonucleoprotein complex containing a box C/D type RNA that is involved in pre-rRNA cleavage. Relationships: is a type of GO:0170049 References: PMID:15367679, PMID:28505386, PMID:30254138